{
  "gene": "UniProtKB:Q9NTJ3",
  "gene_symbol": "SMC4",
  "term_label": "mitotic chromosome condensation",
  "gene_name": "Structural maintenance of chromosomes protein 4",
  "term_id": "GO:0007076"
}